transforming growth factor beta receptor activity, type III [GO:0070123] (molecular function) Relationships: is a type of transforming growth factor beta receptor activity [GO:0005024] References: PMID:9759503 Sources: GOC:BHF, GOC:mah Definition: Combining with transforming growth factor beta to initiate a change in cell activity; facilitates ligand binding to type I and type II TGF-beta receptors. Also known as: type III TGF-beta receptor activity, type III TGFbeta receptor activity, type III transforming growth factor beta receptor activity, betaglycan, endoglin, transforming growth factor beta ligand binding to type III receptor